{
  "gene_name": "DENN domain-containing protein 4C",
  "term_label": "guanyl-nucleotide exchange factor activity",
  "term_id": "GO:0005085",
  "gene_symbol": "DENND4C",
  "gene": "UniProtKB:Q5VZ89"
}